{
  "gene": "UniProtKB:O94900",
  "gene_symbol": "TOX",
  "gene_name": "Thymocyte selection-associated high mobility group box protein TOX",
  "term_label": "leukocyte differentiation",
  "term_id": "GO:0002521"
}